{
  "term_id": "UNKNOWN:0002",
  "gene_name": "Small cysteine and glycine repeat-containing protein 5",
  "gene": "UniProtKB:A0A286YF46",
  "gene_symbol": "SCYGR5",
  "term_label": "Unknown biological process"
}